2-deoxyglucosidase activity [GO:0047539] (molecular function) Definition: Catalysis of the reaction: H2O + a 2-deoxy-alpha-D-glucoside = 2-deoxy-D-glucose + an alcohol. Sources: EC:3.2.1.112, MetaCyc:2-DEOXYGLUCOSIDASE-RXN Also known as: 2-deoxy-alpha-D-glucosidase activity, 2-deoxy-alpha-D-glucoside deoxyglucohydrolase activity, 2-deoxy-alpha-glucosidase activity Relationships: is a type of GO:0015926